{
  "term_label": "Unknown biological process",
  "gene": "UniProtKB:Q9H7Z7",
  "gene_symbol": "PTGES2",
  "term_id": "UNKNOWN:0002",
  "gene_name": "Prostaglandin E synthase 2"
}